{
  "term_label": "hair cycle",
  "gene": "UniProtKB:A0A140TA64",
  "gene_symbol": "LOC100996750",
  "gene_name": "Uncharacterized protein",
  "term_id": "GO:0042633"
}